{
  "gene_name": "Putative golgin subfamily A member 8F_8G",
  "gene": "UniProtKB:Q08AF8",
  "gene_symbol": "GOLGA8G",
  "term_id": "UNKNOWN:0001",
  "term_label": "Unknown molecular function"
}